{
  "gene_symbol": "WDR97",
  "term_label": "Unknown cellular component",
  "gene_name": "WD repeat-containing protein 97",
  "gene": "UniProtKB:A6NE52",
  "term_id": "UNKNOWN:0003"
}